transcription initiation-coupled chromatin remodeling [GO:0045815] (biological process) References: PMID:34414474 Definition: An epigenetic mechanism of regulation of gene expression that involves chromatin remodeling to capacitate gene expression by either modifying the chromatin fiber, the nucleosomal histones, or the DNA. Relationships: is a type of GO:0141137; is part of transcription initiation at RNA polymerase II promoter [GO:0006367] Note: This regulation is exemplified by members of the trithorax group, which maintain the active state of homeotic gene transcription. Do not confuse with GO:0140673 ; transcriptional elongation-coupled chromatin remodeling, which describes the reforming of chromatin after RNA polymerase II passage. Regulation: negatively regulated by negative regulation of transcription initiation-coupled chromatin remodeling [GO:0160217] Also known as: chromatin-mediated maintenance of transcription, epigenetic maintenance of chromatin in transcription-competent conformation, maintenance of chromatin in transcription-competent conformation, transciptional initiation-coupled chromatin remodeling, transcription initiation coupled chromatin remodeling, transcription initiation coupled chromatin remodelling, transcriptional initiation-coupled chromatin remodeling, transcriptional initiation-coupled chromatin remodelling, DNA replication-independent chromatin organization, euchromatin assembly, euchromatin organisation, euchromatin organization, long-term maintenance of gene activation Subtypes: GO:0044029